all-trans-retinyl-palmitate hydrolase, 11-cis retinol forming activity [GO:0052884] (molecular function) Sources: RHEA:31775 Definition: Catalysis of the reaction: H2O + all-trans-retinyl palmitate = 11-cis-retinol + H+ + palmitate. Also known as: all-trans-retinol isomerase:hydrolase activity, all-trans-retinyl-palmitate hydrolase activity, retinoid isomerohydrolase activity, retinol isomerase activity Relationships: is_a retinyl-palmitate esterase activity [GO:0050253]